{
  "term_label": "cyclic-GMP-AMP transmembrane import across plasma membrane",
  "gene_symbol": "LRRC8C",
  "term_id": "GO:0140361",
  "gene_name": "Volume-regulated anion channel subunit LRRC8C",
  "gene": "UniProtKB:Q8TDW0"
}